branched-chain amino acid biosynthetic process [GO:0009082] (biological process) Also known as: branched chain family amino acid anabolism, branched chain family amino acid biosynthesis, branched chain family amino acid biosynthetic process, branched chain family amino acid formation, branched chain family amino acid synthesis Subtypes: isoleucine biosynthetic process [GO:0009097], L-leucine biosynthetic process [GO:0009098], L-valine biosynthetic process [GO:0009099], D-leucine biosynthetic process [GO:1900833] Relationships: is a type of branched-chain amino acid metabolic process [GO:0009081]; is a type of carboxylic acid biosynthetic process [GO:0046394] Sources: GOC:ai Definition: The chemical reactions and pathways resulting in the formation of amino acids containing a branched carbon skeleton, comprising isoleucine, leucine and valine.